{
  "term_label": "Unknown molecular function",
  "term_id": "UNKNOWN:0001",
  "gene_symbol": "INO80D",
  "gene": "UniProtKB:Q53TQ3",
  "gene_name": "INO80 complex subunit D"
}